{
  "gene_symbol": "ABCD2",
  "term_label": "peroxisome organization",
  "term_id": "GO:0007031",
  "gene": "UniProtKB:Q9UBJ2",
  "gene_name": "ATP-binding cassette sub-family D member 2"
}